{
  "gene": "UniProtKB:P0C024",
  "term_id": "GO:0010945",
  "gene_name": "Peroxisomal coenzyme A diphosphatase NUDT7",
  "term_label": "coenzyme A diphosphatase activity",
  "gene_symbol": "NUDT7"
}